cellular response to disaccharide stimulus [GO:0071324] (biological process) Relationships: is a type of GO:0034285; is a type of GO:0071322 Subtypes: cellular response to trehalose stimulus [GO:0071327], cellular response to maltose stimulus [GO:0071328], cellular response to sucrose stimulus [GO:0071329], cellular response to trehalose-6-phosphate stimulus [GO:0071330] Definition: Any process that results in a change in state or activity of a cell (in terms of movement, secretion, enzyme production, gene expression, etc.) as a result of a disaccharide stimulus. Sources: GOC:mah